{
  "gene_name": "Heart- and neural crest derivatives-expressed protein 1",
  "term_id": "GO:0007507",
  "gene_symbol": "HAND1",
  "term_label": "heart development",
  "gene": "UniProtKB:O96004"
}